{
  "term_id": "GO:0007156",
  "gene": "UniProtKB:Q02246",
  "gene_name": "Contactin-2",
  "gene_symbol": "CNTN2",
  "term_label": "homophilic cell-cell adhesion"
}